{
  "gene": "UniProtKB:P0DJ93",
  "term_id": "UNKNOWN:0003",
  "gene_symbol": "SMIM13",
  "gene_name": "Small integral membrane protein 13",
  "term_label": "Unknown cellular component"
}